{
  "term_label": "neuropeptide signaling pathway",
  "term_id": "GO:0007218",
  "gene_name": "Melanin-concentrating hormone receptor 2",
  "gene": "UniProtKB:Q969V1",
  "gene_symbol": "MCHR2"
}